{
  "gene_name": "Hemopexin",
  "gene_symbol": "HPX",
  "gene": "UniProtKB:P02790",
  "term_id": "GO:0005615",
  "term_label": "extracellular space"
}